{
  "gene": "UniProtKB:Q8NGX5",
  "term_label": "membrane",
  "gene_name": "Olfactory receptor 10K1",
  "gene_symbol": "OR10K1",
  "term_id": "GO:0016020"
}